{
  "gene_symbol": "MOB3C",
  "gene": "UniProtKB:Q70IA8",
  "term_label": "signal transduction",
  "term_id": "GO:0007165",
  "gene_name": "MOB kinase activator 3C"
}